{
  "term_id": "GO:0005524",
  "term_label": "ATP binding",
  "gene_symbol": "HSP90AB4P",
  "gene_name": "Putative heat shock protein HSP 90-beta 4",
  "gene": "UniProtKB:Q58FF6"
}